{
  "gene": "UniProtKB:P04899",
  "term_id": "GO:0031683",
  "gene_name": "Guanine nucleotide-binding protein G(i) subunit alpha-2",
  "gene_symbol": "GNAI2",
  "term_label": "G-protein beta/gamma-subunit complex binding"
}